{
  "term_id": "GO:0005262",
  "gene_symbol": "PKDREJ",
  "gene_name": "Polycystin family receptor for egg jelly",
  "term_label": "calcium channel activity",
  "gene": "UniProtKB:Q9NTG1"
}